{
  "term_id": "UNKNOWN:0001",
  "gene": "UniProtKB:Q9UKN8",
  "term_label": "Unknown molecular function",
  "gene_symbol": "GTF3C4",
  "gene_name": "General transcription factor 3C polypeptide 4"
}